regulation of Schwann cell chemotaxis [GO:1904266] (biological process) Subtypes: GO:1904267, positive regulation of Schwann cell chemotaxis [GO:1904268] Relationships: is a type of regulation of chemotaxis [GO:0050920]; is a type of GO:1900147; regulates GO:1990751 Definition: Any process that modulates the frequency, rate or extent of Schwann cell chemotaxis. References: PMID:16203995 Sources: GOC:TermGenie, GO_REF:0000058